{
  "term_id": "GO:0003725",
  "gene": "UniProtKB:Q9Y6K5",
  "term_label": "double-stranded RNA binding",
  "gene_symbol": "OAS3",
  "gene_name": "2'-5'-oligoadenylate synthase 3"
}